regulation of branching involved in prostate gland morphogenesis [GO:0060687] (biological process) Definition: Any process that modulates the rate, frequency, or extent of prostate gland branching, the process in which the branching structure of the prostate gland is generated and organized. A branch is a division or offshoot from a main stem. Relationships: is a type of regulation of morphogenesis of a branching structure [GO:0060688]; is a type of regulation of morphogenesis of an epithelium [GO:1905330]; is a type of regulation of reproductive process [GO:2000241]; regulates GO:0060442 Sources: GOC:dph